{
  "gene": "UniProtKB:P49674",
  "term_label": "nucleus",
  "gene_name": "Casein kinase I isoform epsilon",
  "gene_symbol": "CSNK1E",
  "term_id": "GO:0005634"
}